{
  "term_id": "GO:0035861",
  "gene": "UniProtKB:Q86V20",
  "term_label": "site of double-strand break",
  "gene_symbol": "SHLD2",
  "gene_name": "Shieldin complex subunit 2"
}